P450-containing electron transport chain [GO:0140647] (biological process) Relationships: is a type of GO:0022900 References: PMID:16042601 Definition: A electron transport chain in which one or more electron carriers operate to transfer electrons from donors to a cytochrome P450 protein or domain. Electron carriers operating in this chain include FAD-containing flavoproteins or domains, FMN domains, ferredoxins and cytochrome b5. The reduced cytochrome P450 functions as the terminal oxidase and participates in a wide range of biochemical pathways. Also known as: P450-containing system